negative regulation of presynaptic active zone assembly [GO:1905519] (biological process) References: PMID:15797875 Sources: GOC:BHF, GOC:TermGenie, GOC:rl, GO_REF:0000058 Relationships: is_a regulation of presynaptic active zone assembly [GO:1905518]; is a type of negative regulation of presynapse assembly [GO:1905607]; negatively regulates presynaptic active zone assembly [GO:1904071] Definition: Any process that stops, prevents or reduces the frequency, rate or extent of presynaptic active zone assembly. Also known as: down regulation of pre-synaptic active zone assembly, down regulation of pre-synaptic active zone formation, down regulation of presynaptic active zone assembly, down regulation of presynaptic active zone formation, down-regulation of pre-synaptic active zone assembly, down-regulation of pre-synaptic active zone formation, down-regulation of presynaptic active zone assembly, down-regulation of presynaptic active zone formation, downregulation of pre-synaptic active zone assembly, downregulation of pre-synaptic active zone formation, downregulation of presynaptic active zone assembly, downregulation of presynaptic active zone formation, negative regulation of pre-synaptic active zone assembly, negative regulation of pre-synaptic active zone formation, negative regulation of presynaptic active zone formation, down regulation of pre-synaptic active zone component assembly, down regulation of pre-synaptic active zone component formation, down-regulation of pre-synaptic active zone component assembly, down-regulation of pre-synaptic active zone component formation, downregulation of pre-synaptic active zone component assembly, downregulation of pre-synaptic active zone component formation, inhibition of pre-synaptic active zone assembly, inhibition of pre-synaptic active zone component assembly, inhibition of pre-synaptic active zone component formation, inhibition of pre-synaptic active zone formation, inhibition of presynaptic active zone assembly, inhibition of presynaptic active zone formation, negative regulation of pre-synaptic active zone component assembly, negative regulation of pre-synaptic active zone component formation